{
  "gene_name": "Serine_threonine-protein phosphatase 1 regulatory subunit 10",
  "term_label": "PTW/PP1 phosphatase complex",
  "gene_symbol": "PPP1R10",
  "gene": "UniProtKB:Q96QC0",
  "term_id": "GO:0072357"
}